insecticide catabolic process [GO:0046701] (biological process) Relationships: is a type of toxin catabolic process [GO:0009407]; is a type of GO:0017143; is a type of xenobiotic catabolic process [GO:0042178] Also known as: insecticide breakdown, insecticide catabolism, insecticide degradation Sources: GOC:ai Subtypes: 1,1,1-trichloro-2,2-bis-(4-chlorophenyl)ethane catabolic process [GO:0042188] Definition: The chemical reactions and pathways resulting in the breakdown of insecticides, chemicals used to kill insects.